positive regulation of anterior head development [GO:2000744] (BP) Relationships: is a type of positive regulation of developmental process [GO:0051094]; is a type of regulation of anterior head development [GO:2000742]; positively regulates anterior head development [GO:0097065] Sources: GOC:obol Definition: Any process that activates or increases the frequency, rate or extent of anterior head development.